{
  "gene_symbol": "TMT1B",
  "gene_name": "Thiol S-methyltransferase TMT1B",
  "term_label": "Unknown biological process",
  "term_id": "UNKNOWN:0002",
  "gene": "UniProtKB:Q6UX53"
}